{
  "gene_symbol": "MTMR8",
  "term_id": "GO:0005635",
  "gene": "UniProtKB:Q96EF0",
  "gene_name": "Myotubularin-related protein 8",
  "term_label": "nuclear envelope"
}